peptide antigen assembly with MHC class I protein complex [GO:0002502] (biological process) Relationships: is a type of peptide antigen assembly with MHC protein complex [GO:0002501]; is part of GO:0002397; is part of antigen processing and presentation of peptide antigen via MHC class I [GO:0002474] Definition: The binding of a peptide to the antigen binding groove of an MHC class I protein complex. Class I here refers to classical class I molecules. References: PMID:15771591 Sources: GOC:add, ISBN:0781735149